{
  "gene_symbol": "PLXDC1",
  "gene_name": "Plexin domain-containing protein 1",
  "gene": "UniProtKB:Q8IUK5",
  "term_id": "UNKNOWN:0003",
  "term_label": "Unknown cellular component"
}